alkylglycerol kinase activity [GO:0047649] (molecular function) Definition: Catalysis of the reaction: 1-alkyl-sn-glycerol + ATP = 1-alkyl-sn-glycerol 3-phosphate + ADP + 2 H+. Also known as: 1-alkylglycerol kinase (phosphorylating), ATP-alkylglycerol phosphotransferase activity, ATP:1-O-alkyl-sn-glycerol 3-phosphotransferase activity, ATP:1-alkyl-sn-glycerol phosphotransferase activity, alkylglycerol phosphotransferase activity Relationships: is a type of kinase activity [GO:0016301]; is a type of GO:0016773 Sources: EC:2.7.1.93, RHEA:16937